{
  "term_id": "UNKNOWN:0003",
  "term_label": "Unknown cellular component",
  "gene": "UniProtKB:Q7RTV5",
  "gene_symbol": "PRXL2C",
  "gene_name": "Peroxiredoxin-like 2C"
}